{
  "gene_name": "Inactive tyrosine-protein kinase PEAK1",
  "gene": "UniProtKB:Q9H792",
  "term_label": "actin cytoskeleton",
  "term_id": "GO:0015629",
  "gene_symbol": "PEAK1"
}